{
  "term_label": "Unknown biological process",
  "term_id": "UNKNOWN:0002",
  "gene_symbol": "PRO1854",
  "gene": "UniProtKB:Q9UHT4",
  "gene_name": "Putative uncharacterized protein PRO1854"
}